{
  "gene_name": "Potassium voltage-gated channel subfamily G member 1",
  "gene": "UniProtKB:Q9UIX4",
  "gene_symbol": "KCNG1",
  "term_label": "voltage-gated potassium channel complex",
  "term_id": "GO:0008076"
}